{
  "gene": "UniProtKB:P08559",
  "term_label": "pyruvate decarboxylation to acetyl-CoA",
  "gene_symbol": "PDHA1",
  "term_id": "GO:0006086",
  "gene_name": "Pyruvate dehydrogenase E1 component subunit alpha, somatic form, mitochondrial"
}